{
  "gene": "UniProtKB:Q9UNW1",
  "term_label": "acid phosphatase activity",
  "term_id": "GO:0003993",
  "gene_name": "Multiple inositol polyphosphate phosphatase 1",
  "gene_symbol": "MINPP1"
}